{
  "term_label": "eukaryotic translation initiation factor 3 complex, eIF3e",
  "term_id": "GO:0071540",
  "gene_name": "Eukaryotic translation initiation factor 3 subunit A",
  "gene_symbol": "EIF3A",
  "gene": "UniProtKB:Q14152"
}